{
  "term_label": "nucleus",
  "gene_name": "Elongator complex protein 5",
  "gene_symbol": "ELP5",
  "gene": "UniProtKB:Q8TE02",
  "term_id": "GO:0005634"
}